{
  "gene_symbol": "CDC25A",
  "term_label": "G2/M transition of mitotic cell cycle",
  "gene": "UniProtKB:P30304",
  "term_id": "GO:0000086",
  "gene_name": "M-phase inducer phosphatase 1"
}